{
  "term_label": "protein-succinyllysine desuccinylase activity",
  "gene_symbol": "SIRT5",
  "term_id": "GO:0036055",
  "gene": "UniProtKB:Q9NXA8",
  "gene_name": "NAD-dependent protein deacylase sirtuin-5, mitochondrial"
}